{
  "gene": "UniProtKB:Q9HCK8",
  "term_id": "GO:0007420",
  "gene_name": "Chromodomain-helicase-DNA-binding protein 8",
  "term_label": "brain development",
  "gene_symbol": "CHD8"
}